{
  "term_label": "regulation of mRNA splicing, via spliceosome",
  "term_id": "GO:0048024",
  "gene_symbol": "HNRNPK",
  "gene_name": "Heterogeneous nuclear ribonucleoprotein K",
  "gene": "UniProtKB:P61978"
}